{
  "gene": "UniProtKB:P17097",
  "term_label": "RNA polymerase II cis-regulatory region sequence-specific DNA binding",
  "term_id": "GO:0000978",
  "gene_symbol": "ZNF7",
  "gene_name": "Zinc finger protein 7"
}